{
  "term_label": "Unknown biological process",
  "gene": "UniProtKB:Q5TG53",
  "term_id": "UNKNOWN:0002",
  "gene_name": "Putative uncharacterized protein SERTAD4-AS1",
  "gene_symbol": "SERTAD4-AS1"
}